{
  "gene_symbol": "DPH1",
  "term_id": "GO:0017183",
  "term_label": "protein histidyl modification to diphthamide",
  "gene_name": "2-(3-amino-3-carboxypropyl)histidine synthase subunit 1",
  "gene": "UniProtKB:Q9BZG8"
}